granulocyte macrophage colony-stimulating factor receptor activity [GO:0004901] (molecular function) Also known as: CSF-2 receptor activity, GM-CSF receptor activity, GMC-SF receptor activity, granulocyte macrophage colony stimulating factor receptor activity, CSF2R Relationships: is_a GO:0004896; is part of GO:0038157; has part GO:0042021 Definition: Combining with granulocyte macrophage colony-stimulating factor (GM-CSF) and transmitting the signal from one side of the membrane to the other to initiate a change in cell activity. Sources: GOC:mah, GOC:signaling